{
  "term_id": "GO:0030198",
  "gene": "UniProtKB:Q8TB73",
  "gene_symbol": "NDNF",
  "gene_name": "Protein NDNF",
  "term_label": "extracellular matrix organization"
}